{
  "gene_symbol": "HSPE1",
  "term_id": "GO:0051082",
  "gene": "UniProtKB:P61604",
  "term_label": "unfolded protein binding",
  "gene_name": "10 kDa heat shock protein, mitochondrial"
}